negative regulation of defecation rhythm [GO:2000747] (biological process) Definition: Any process that stops, prevents or reduces the frequency, rate or extent of defecation rhythm. Sources: GOC:kmv Relationships: is a type of negative regulation of defecation [GO:2000293]; is a type of regulation of defecation rhythm [GO:2000746]; negatively regulates defecation rhythm [GO:0035882] Also known as: negative regulation of DMP, negative regulation of defecation cycle, negative regulation of defecation motor program, negative regulation of defecation behavior